ribonuclease MRP activity [GO:0000171] (molecular function) Relationships: is a type of RNA endonuclease activity [GO:0004521]; is a type of GO:0016788 References: PMID:17881380 Definition: Catalysis of the site-specific cleavage of RNA by a catalytic RNA-mediated mechanism; substrates include the A3 site in the ITS1 of pre-rRNA. Also known as: RNase MRP